sensory organ development [GO:0007423] (biological process) Subtypes: eye development [GO:0001654], amphid sensory organ development [GO:0003386], ocellus development [GO:0008056], chaeta development [GO:0022416], GO:0043583, nose development [GO:0043584], tongue development [GO:0043586], GO:0045498, neuromast development [GO:0048884], taste bud development [GO:0061193], GO:0071599 Also known as: sense organ development Relationships: is a type of animal organ development [GO:0048513] Definition: The process whose specific outcome is the progression of sensory organs over time, from its formation to the mature structure. Sources: GOC:go_curators